{
  "gene": "UniProtKB:O15041",
  "term_label": "semaphorin-plexin signaling pathway",
  "term_id": "GO:0071526",
  "gene_symbol": "SEMA3E",
  "gene_name": "Semaphorin-3E"
}